{
  "gene_symbol": "KMT2E",
  "term_label": "Set3 complex",
  "term_id": "GO:0034967",
  "gene": "UniProtKB:Q8IZD2",
  "gene_name": "Inactive histone-lysine N-methyltransferase 2E"
}